{
  "term_label": "rRNA methylation",
  "gene_symbol": "NSUN3",
  "gene_name": "tRNA (cytosine(34)-C(5))-methyltransferase, mitochondrial",
  "term_id": "GO:0031167",
  "gene": "UniProtKB:Q9H649"
}